negative regulation of innate immune response [GO:0045824] (biological process) Also known as: down regulation of innate immune response, down-regulation of innate immune response, downregulation of innate immune response, inhibition of innate immune response Sources: GOC:go_curators Relationships: is a type of GO:0002832; is a type of negative regulation of defense response [GO:0031348]; is a type of negative regulation of response to external stimulus [GO:0032102]; is a type of regulation of innate immune response [GO:0045088]; is a type of negative regulation of immune response [GO:0050777]; negatively regulates innate immune response [GO:0045087] Definition: Any process that stops, prevents, or reduces the frequency, rate or extent of the innate immune response. Subtypes: negative regulation of complement activation, lectin pathway [GO:0001869], negative regulation of natural killer cell mediated immunity [GO:0002716], negative regulation of plant-type hypersensitive response [GO:0034051], negative regulation of melanization defense response [GO:0035009], GO:0045957, negative regulation of respiratory burst involved in inflammatory response [GO:0060266], negative regulation of response to type II interferon [GO:0060331], negative regulation of type I interferon-mediated signaling pathway [GO:0060339], negative regulation of age-related resistance [GO:1904249], negative regulation of antifungal innate immune response [GO:1905035], negative regulation of innate immunity memory response [GO:1905681]